{
  "gene_name": "POTE ankyrin domain family member D",
  "gene": "UniProtKB:Q86YR6",
  "gene_symbol": "POTED",
  "term_id": "UNKNOWN:0001",
  "term_label": "Unknown molecular function"
}